{
  "gene": "UniProtKB:Q96N67",
  "term_id": "GO:0005085",
  "gene_symbol": "DOCK7",
  "gene_name": "Dedicator of cytokinesis protein 7",
  "term_label": "guanyl-nucleotide exchange factor activity"
}